{
  "gene_name": "Protein ANKUB1",
  "term_id": "UNKNOWN:0001",
  "gene_symbol": "ANKUB1",
  "term_label": "Unknown molecular function",
  "gene": "UniProtKB:A6NFN9"
}